{
  "term_label": "Unknown cellular component",
  "gene": "UniProtKB:Q8N9G6",
  "term_id": "UNKNOWN:0003",
  "gene_name": "Putative UPF0607 protein FLJ37424",
  "gene_symbol": "Q8N9G6"
}